type B gastrin/cholecystokinin receptor binding [GO:0031741] (molecular function) Also known as: type B gastrin/cholecystokinin receptor ligand Definition: Binding to a type B gastrin/cholecystokinin receptor. Sources: GOC:mah, GOC:nln Relationships: is a type of GO:0031739